oligosaccharyltransferase complex binding [GO:0062062] (MF) Definition: Binding to an oligosaccharyltransferase complex. References: PMID:12887896 Relationships: is a type of protein-containing complex binding [GO:0044877]